{
  "gene_name": "Methyl-CpG-binding domain protein 2",
  "gene": "UniProtKB:Q9UBB5",
  "term_id": "GO:0006346",
  "gene_symbol": "MBD2",
  "term_label": "DNA methylation-dependent constitutive heterochromatin formation"
}